{
  "gene": "UniProtKB:Q9NU23",
  "gene_name": "LYR motif-containing protein 2",
  "term_id": "GO:0005739",
  "term_label": "mitochondrion",
  "gene_symbol": "LYRM2"
}